{
  "gene_name": "T cell receptor beta variable 4-2",
  "term_id": "UNKNOWN:0001",
  "gene": "UniProtKB:A0A539",
  "term_label": "Unknown molecular function",
  "gene_symbol": "TRBV4-2"
}